{
  "gene_name": "Oxysterol-binding protein 1",
  "gene": "UniProtKB:P22059",
  "term_id": "GO:0097038",
  "term_label": "perinuclear endoplasmic reticulum",
  "gene_symbol": "OSBP"
}